{
  "term_id": "GO:0005737",
  "gene_name": "Myotubularin-related protein 2",
  "gene": "UniProtKB:Q13614",
  "gene_symbol": "MTMR2",
  "term_label": "cytoplasm"
}